{
  "term_id": "GO:0004252",
  "term_label": "serine-type endopeptidase activity",
  "gene_name": "Kallikrein-2",
  "gene_symbol": "KLK2",
  "gene": "UniProtKB:P20151"
}